alpha9-beta1 integrin-osteopontin complex [GO:0071127] (cellular component) References: PMID:16005200 Definition: A protein complex that consists of an alpha9-beta1 integrin complex bound to osteopontin. Also known as: ITGA9-ITGB1-SPP1 complex Relationships: is a type of plasma membrane protein complex [GO:0098797]